{
  "term_label": "succinate-CoA ligase complex",
  "gene_name": "Succinate--CoA ligase [GDP-forming] subunit beta, mitochondrial",
  "term_id": "GO:0042709",
  "gene": "UniProtKB:Q96I99",
  "gene_symbol": "SUCLG2"
}